phytyl diphosphate biosynthetic process [GO:0033521] (biological process) Also known as: phytyl diphosphate anabolism, phytyl diphosphate biosynthesis, phytyl diphosphate formation, phytyl diphosphate synthesis Definition: The chemical reactions and pathways resulting in the formation of phytyl diphosphate, (2E)-3,7,11,15-tetramethylhexadec-2-en-1-yl trihydrogen diphosphate. Relationships: is a type of phospholipid biosynthetic process [GO:0008654]; is a type of terpenoid biosynthetic process [GO:0016114] Sources: GOC:mah